detection of cell density [GO:0060245] (BP) Relationships: is a type of detection of biotic stimulus [GO:0009595] Subtypes: quorum sensing [GO:0009372], contact inhibition [GO:0060242] Definition: The series of events in which information about the density of cells in a population is received and converted into a molecular signal. Sources: GOC:dph